{
  "gene_symbol": "KLRG2",
  "term_id": "UNKNOWN:0002",
  "term_label": "Unknown biological process",
  "gene": "UniProtKB:A4D1S0",
  "gene_name": "Killer cell lectin-like receptor subfamily G member 2"
}